{
  "term_id": "GO:0032391",
  "gene_name": "Protein fantom",
  "term_label": "photoreceptor connecting cilium",
  "gene_symbol": "RPGRIP1L",
  "gene": "UniProtKB:Q68CZ1"
}